regulation of beta 2 integrin biosynthetic process [GO:0045115] (biological process) Definition: Any process that modulates the frequency, rate or extent of the chemical reactions and pathways resulting in the formation of beta 2 integrins. Sources: GOC:go_curators Relationships: is a type of regulation of integrin biosynthetic process [GO:0045113]; regulates beta 2 integrin biosynthetic process [GO:0045114] Also known as: regulation of beta 2 integrin anabolism, regulation of beta 2 integrin biosynthesis, regulation of beta 2 integrin formation, regulation of beta 2 integrin synthesis Subtypes: negative regulation of beta 2 integrin biosynthetic process [GO:0045774], positive regulation of beta 2 integrin biosynthetic process [GO:0045775]